{
  "gene_symbol": "PPP3R2",
  "term_label": "calcineurin complex",
  "gene_name": "Calcineurin subunit B type 2",
  "term_id": "GO:0005955",
  "gene": "UniProtKB:Q96LZ3"
}